negative regulation of epithelial cell differentiation [GO:0030857] (biological process) Definition: Any process that stops, prevents, or reduces the frequency, rate or extent of epithelial cell differentiation. Sources: GOC:mah Relationships: is a type of regulation of epithelial cell differentiation [GO:0030856]; is a type of negative regulation of cell differentiation [GO:0045596]; negatively regulates epithelial cell differentiation [GO:0030855] Subtypes: inhibition of neuroepithelial cell differentiation [GO:0002085], negative regulation of polarized epithelial cell differentiation [GO:0030861], GO:0045593, negative regulation of endothelial cell differentiation [GO:0045602], negative regulation of epidermal cell differentiation [GO:0045605], negative regulation of hepatocyte differentiation [GO:0070367], GO:1901247, negative regulation of lung goblet cell differentiation [GO:1901250], GO:1902747, negative regulation of establishment of Sertoli cell barrier [GO:1904445], GO:1905299, negative regulation of pancreatic A cell differentiation [GO:2000227], GO:2000697 Also known as: down regulation of epithelial cell differentiation, down-regulation of epithelial cell differentiation, downregulation of epithelial cell differentiation, inhibition of epithelial cell differentiation